{
  "gene": "UniProtKB:Q8IZF2",
  "term_label": "glucose homeostasis",
  "gene_name": "Adhesion G protein-coupled receptor F5",
  "term_id": "GO:0042593",
  "gene_symbol": "ADGRF5"
}